hexose import across plasma membrane [GO:0140271] (biological process) Definition: The directed movement of hexose from outside of a cell, across the plasma membrane and into the cytosol. References: PMID:10735857 Relationships: is a type of hexose transmembrane transport [GO:0008645]; is a type of carbohydrate import across plasma membrane [GO:0098704] Subtypes: D-glucose import across plasma membrane [GO:0098708], galactose import across plasma membrane [GO:0140425], fructose import across plasma membrane [GO:1990539]